{
  "term_label": "mitochondrion",
  "gene": "UniProtKB:Q9NXA8",
  "gene_symbol": "SIRT5",
  "gene_name": "NAD-dependent protein deacylase sirtuin-5, mitochondrial",
  "term_id": "GO:0005739"
}